netrin receptor activity involved in chemoattraction [GO:0038006] (molecular function) Relationships: is a type of netrin receptor activity [GO:0005042]; BFO_0000050 GO:0050918 Definition: Combining with a netrin signal and transmitting the signal from one side of the membrane to the other to contribute to the directed movement of a motile cell towards a higher concentration of netrin. Also known as: attractive netrin receptor activity, netrin receptor activity involved in positive chemotaxis Sources: GOC:signaling